{
  "gene_name": "NHP2-like protein 1",
  "gene_symbol": "SNU13",
  "term_id": "GO:0000398",
  "gene": "UniProtKB:P55769",
  "term_label": "mRNA splicing, via spliceosome"
}